{
  "term_id": "GO:0051017",
  "gene_name": "Espin-like protein",
  "gene": "UniProtKB:Q6ZVH7",
  "term_label": "actin filament bundle assembly",
  "gene_symbol": "ESPNL"
}